{
  "term_id": "GO:0044325",
  "term_label": "transmembrane transporter binding",
  "gene": "UniProtKB:Q9UJ90",
  "gene_symbol": "KCNE5",
  "gene_name": "Potassium voltage-gated channel subfamily E regulatory beta subunit 5"
}